{
  "term_label": "phosphocreatine biosynthetic process",
  "gene_symbol": "CKM",
  "gene": "UniProtKB:P06732",
  "gene_name": "Creatine kinase M-type",
  "term_id": "GO:0046314"
}